{
  "term_label": "adaptive immune response",
  "term_id": "GO:0002250",
  "gene_name": "Interleukin-18 receptor 1",
  "gene": "UniProtKB:Q13478",
  "gene_symbol": "IL18R1"
}